{
  "gene": "UniProtKB:Q9NZM1",
  "term_label": "calcium ion binding",
  "gene_symbol": "MYOF",
  "gene_name": "Myoferlin",
  "term_id": "GO:0005509"
}